{
  "gene_symbol": "SLC22A31",
  "term_id": "UNKNOWN:0002",
  "gene_name": "Putative solute carrier family 22 member 31",
  "gene": "UniProtKB:A6NKX4",
  "term_label": "Unknown biological process"
}